methyl-CpNpG binding [GO:0010428] (molecular function) Relationships: is a type of GO:0000166 Definition: Binding to a methylated cytosine/unspecified/guanine trinucleotide. References: PMID:17239600